{
  "gene": "UniProtKB:Q9NXJ0",
  "gene_name": "Membrane-spanning 4-domains subfamily A member 12",
  "term_id": "GO:0007166",
  "gene_symbol": "MS4A12",
  "term_label": "cell surface receptor signaling pathway"
}